{
  "gene_name": "Leiomodin-1",
  "gene_symbol": "LMOD1",
  "gene": "UniProtKB:P29536",
  "term_label": "tropomyosin binding",
  "term_id": "GO:0005523"
}